{
  "term_label": "extracellular space",
  "gene": "UniProtKB:P0CW18",
  "term_id": "GO:0005615",
  "gene_symbol": "PRSS56",
  "gene_name": "Serine protease 56"
}